pronephric nephron tubule epithelial cell differentiation [GO:0035778] (biological process) Relationships: is_a cell differentiation involved in pronephros development [GO:0039014]; is a type of nephron tubule epithelial cell differentiation [GO:0072160]; is part of pronephric nephron tubule development [GO:0039020] References: PMID:18787069 Sources: GOC:mtg_kidney_jan10, GOC:yaf Definition: The process in which relatively unspecialized cells acquire specialized structural and/or functional features that characterize the cells of the pronephric nephron tubule as it progresses from its formation to the mature state.